positive regulation of macrophage inflammatory protein 1 alpha production [GO:0071642] (biological process) Definition: Any process that activates or increases the frequency, rate, or extent of production of macrophage inflammatory protein 1 alpha. Sources: GOC:mah Also known as: positive regulation of macrophage inflammatory protein production, positive regulation of CCL3 production, positive regulation of MIP-1a production, positive regulation of chemokine (C-C motif) ligand 3 production Relationships: is a type of positive regulation of chemokine production [GO:0032722]; is a type of regulation of macrophage inflammatory protein 1 alpha production [GO:0071640]; positively regulates macrophage inflammatory protein-1 alpha production [GO:0071608]